4-nitrotoluene monooxygenase activity [GO:0102037] (molecular function) Definition: Catalysis of the reaction: H+ + 4-nitrotoluene + NADH + O2 = 4-nitrobenzyl alcohol + NAD+ + H2O. Relationships: is a type of oxidoreductase activity, acting on paired donors, with incorporation or reduction of molecular oxygen, NAD(P)H as one donor, and incorporation of one atom of oxygen [GO:0016709] Sources: GOC:pz